{
  "gene_name": "Cullin-9",
  "term_label": "ubiquitin ligase complex scaffold activity",
  "term_id": "GO:0160072",
  "gene_symbol": "CUL9",
  "gene": "UniProtKB:Q8IWT3"
}